{
  "term_label": "cell adhesion",
  "gene_name": "Protocadherin beta-12",
  "gene": "UniProtKB:Q9Y5F1",
  "term_id": "GO:0007155",
  "gene_symbol": "PCDHB12"
}